{
  "term_label": "actin filament binding",
  "term_id": "GO:0051015",
  "gene_symbol": "MYO1H",
  "gene": "UniProtKB:Q8N1T3",
  "gene_name": "Unconventional myosin-Ih"
}